{
  "gene_name": "CMT1A duplicated region transcript 15 protein",
  "term_id": "UNKNOWN:0003",
  "gene": "UniProtKB:Q96T59",
  "term_label": "Unknown cellular component",
  "gene_symbol": "CDRT15"
}